{
  "gene_symbol": "UGT2B10",
  "gene": "UniProtKB:P36537",
  "term_id": "GO:0008210",
  "gene_name": "UDP-glucuronosyltransferase 2B10",
  "term_label": "estrogen metabolic process"
}